{
  "gene": "UniProtKB:P09105",
  "term_id": "GO:0031838",
  "term_label": "haptoglobin-hemoglobin complex",
  "gene_symbol": "HBQ1",
  "gene_name": "Hemoglobin subunit theta-1"
}